{
  "gene_symbol": "RC3H2",
  "gene_name": "Roquin-2",
  "term_id": "GO:0003729",
  "gene": "UniProtKB:Q9HBD1",
  "term_label": "mRNA binding"
}